epithelial cell differentiation involved in mammary gland bud morphogenesis [GO:0060643] (biological process) Definition: The process in which a cell of the mammary placode becomes a cell of the mammary gland bud. Sources: GOC:dph Relationships: is a type of mammary gland epithelial cell differentiation [GO:0060644]; is part of mammary gland bud formation [GO:0060615] Subtypes: peripheral mammary gland bud epithelial cell differentiation [GO:0060645], GO:0060646